{
  "gene": "UniProtKB:Q00610",
  "gene_name": "Clathrin heavy chain 1",
  "gene_symbol": "CLTC",
  "term_id": "GO:0045334",
  "term_label": "clathrin-coated endocytic vesicle"
}